{
  "gene_name": "Sorting nexin-5",
  "term_id": "GO:0005768",
  "term_label": "endosome",
  "gene_symbol": "SNX5",
  "gene": "UniProtKB:Q9Y5X3"
}